{
  "gene": "UniProtKB:Q5H9U9",
  "term_label": "cytoplasm",
  "gene_symbol": "DDX60L",
  "gene_name": "Probable ATP-dependent RNA helicase DDX60-like",
  "term_id": "GO:0005737"
}